{
  "gene": "UniProtKB:Q9H582",
  "gene_name": "Zinc finger protein 644",
  "gene_symbol": "ZNF644",
  "term_label": "nucleus",
  "term_id": "GO:0005634"
}